{
  "gene_symbol": "PODXL2",
  "term_label": "Unknown molecular function",
  "gene": "UniProtKB:Q9NZ53",
  "term_id": "UNKNOWN:0001",
  "gene_name": "Podocalyxin-like protein 2"
}